{
  "gene_symbol": "CASP6",
  "term_id": "GO:0006915",
  "gene_name": "Caspase-6",
  "term_label": "apoptotic process",
  "gene": "UniProtKB:P55212"
}